symbiont-mediated suppression of host translation termination [GO:0046773] (biological process) Also known as: suppression by virus of host translation termination, viral inhibition of termination of host cell protein biosynthesis, viral inhibition of termination of host cell protein biosynthetic process, viral suppression of termination by host of host cell protein biosynthesis, viral suppression of termination by host of host cell protein biosynthetic process Sources: ISBN:0781718325 Definition: A process in which a symbiont inhibits or disrupts translation termination of host mRNAs. The host is defined as the larger of the organisms involved in a symbiotic interaction. Relationships: is a type of symbiont-mediated perturbation of host gene expression [GO:0039656]